{
  "term_id": "GO:0005737",
  "gene": "UniProtKB:Q9Y5P6",
  "term_label": "cytoplasm",
  "gene_symbol": "GMPPB",
  "gene_name": "Mannose-1-phosphate guanyltransferase beta"
}